{
  "gene_name": "Golgin subfamily A member 6C",
  "term_label": "cis-Golgi network",
  "term_id": "GO:0005801",
  "gene": "UniProtKB:A6NDK9",
  "gene_symbol": "GOLGA6C"
}